{
  "gene_symbol": "ACSL6",
  "term_id": "GO:0016020",
  "gene_name": "Long-chain-fatty-acid--CoA ligase 6",
  "term_label": "membrane",
  "gene": "UniProtKB:Q9UKU0"
}